resolution of mitotic recombination intermediates [GO:0071140] (biological process) Sources: GOC:elh, GOC:mah, GOC:vw Definition: The cleavage and rejoining of intermediates, mitotic recombination to produce two intact molecules in which genetic material has been exchanged. Relationships: is a type of resolution of DNA recombination intermediates [GO:0071139]; is part of mitotic recombination [GO:0006312]